{
  "term_id": "UNKNOWN:0001",
  "gene_name": "General transcription factor 3C polypeptide 2",
  "gene_symbol": "GTF3C2",
  "gene": "UniProtKB:Q8WUA4",
  "term_label": "Unknown molecular function"
}